{
  "gene_symbol": "EIF4G3",
  "gene_name": "Eukaryotic translation initiation factor 4 gamma 3",
  "term_label": "eukaryotic translation initiation factor 4F complex",
  "term_id": "GO:0016281",
  "gene": "UniProtKB:O43432"
}